response to carbamate [GO:0046681] (biological process) Definition: Any process that results in a change in state or activity of a cell or an organism (in terms of movement, secretion, enzyme production, gene expression, etc.) as a result of a carbamate stimulus. Carbamates are a group of insecticides and parasiticides that act by inhibiting cholinesterase. Sources: ISBN:0721662544 Also known as: carbamate resistance, carbamate susceptibility/resistance Relationships: is a type of GO:0017085; is a type of GO:1901698; is a type of response to oxygen-containing compound [GO:1901700]